antisigma factor binding [GO:0045152] (MF) Definition: Binding to an antisigma factor, a factor which inhibits the ability of the sigma factor to function as a transcriptional initiator. Sources: GOC:mlg Also known as: antisigma factor antagonist activity Relationships: is_a protein binding [GO:0005515]